prostacyclin receptor activity [GO:0016501] (molecular function) Relationships: is a type of prostaglandin receptor activity [GO:0004955] Also known as: PGI(2) receptor activity, prostaglandin I receptor activity, PGI receptor activity Sources: ISBN:0198506732 Definition: Combining with prostacyclin (PGI(2)) to initiate a change in cell activity.